{
  "gene_name": "Endothelin-1 receptor",
  "gene": "UniProtKB:P25101",
  "term_id": "GO:0042310",
  "gene_symbol": "EDNRA",
  "term_label": "vasoconstriction"
}